{
  "gene_name": "Carboxypeptidase B",
  "gene_symbol": "CPB1",
  "term_label": "proteolysis",
  "term_id": "GO:0006508",
  "gene": "UniProtKB:P15086"
}